{
  "term_label": "Unknown biological process",
  "term_id": "UNKNOWN:0002",
  "gene_symbol": "SMIM10L2B",
  "gene": "UniProtKB:P0DMW5",
  "gene_name": "Small integral membrane protein 10-like protein 2B"
}